dolichyl-phosphate alpha-N-acetylglucosaminyltransferase activity [GO:0004166] (molecular function) Definition: Catalysis of the reaction: UDP-N-acetyl-D-glucosamine + dolichyl phosphate = UDP + dolichyl N-acetyl-alpha-D-glucosaminyl phosphate. Sources: EC:2.4.1.153 Also known as: UDP-N-acetyl-D-glucosamine:dolichyl-phosphate alpha-N-acetyl-D-glucosaminyltransferase activity, UDP-N-acetylglucosamine-dolichol phosphate N-acetylglucosaminyltransferase activity, dolichyl phosphate N-acetylglucosaminyltransferase activity, dolichyl phosphate acetylglucosaminyltransferase activity, dolichyl-phosphate N-acetylglucosaminyltransferase activity, dolichyl-phosphate acetylglucosaminyltransferase activity, uridine diphosphoacetylglucosamine-dolichol phosphate acetylglucosaminyltransferase activity Relationships: is a type of acetylglucosaminyltransferase activity [GO:0008375]